{
  "term_label": "dendrite",
  "gene_symbol": "HTR2C",
  "gene_name": "5-hydroxytryptamine receptor 2C",
  "term_id": "GO:0030425",
  "gene": "UniProtKB:P28335"
}